peptidyl-1-thioglycine biosynthetic process from peptidyl-glycine [GO:0018173] (BP) Relationships: is a type of GO:0018201; is a type of modified amino acid biosynthetic process [GO:0042398] Also known as: peptidyl-1-thioglycine anabolism from peptidyl-glycine, peptidyl-1-thioglycine formation from peptidyl-glycine, peptidyl-1-thioglycine synthesis from peptidyl-glycine References: PMID:10660523 Sources: RESID:AA0265 Definition: The chemical reactions and pathways resulting in the formation of peptidyl-1-thioglycine from other compounds, including peptidyl-glycine.